{
  "gene_symbol": "NOMO2",
  "term_id": "UNKNOWN:0001",
  "gene_name": "BOS complex subunit NOMO2",
  "term_label": "Unknown molecular function",
  "gene": "UniProtKB:Q5JPE7"
}